{
  "gene_symbol": "KRTAP4-1",
  "gene_name": "Keratin-associated protein 4-1",
  "term_label": "Unknown cellular component",
  "gene": "UniProtKB:Q9BYQ7",
  "term_id": "UNKNOWN:0003"
}